{
  "term_label": "piecemeal microautophagy of the nucleus",
  "gene": "UniProtKB:Q2TAZ0",
  "gene_name": "Autophagy-related protein 2 homolog A",
  "term_id": "GO:0034727",
  "gene_symbol": "ATG2A"
}